{
  "gene": "UniProtKB:Q8NHB1",
  "gene_symbol": "OR2V1",
  "gene_name": "Olfactory receptor 2V1",
  "term_id": "GO:0004984",
  "term_label": "olfactory receptor activity"
}